{
  "term_label": "Unknown molecular function",
  "gene_name": "Putative uncharacterized protein encoded by LINC02877",
  "term_id": "UNKNOWN:0001",
  "gene": "UniProtKB:P0CE67",
  "gene_symbol": "LINC02877"
}